hemicellulose catabolic process [GO:2000895] (BP) Relationships: is a type of polysaccharide catabolic process [GO:0000272] Regulation: regulated by regulation of hemicellulose catabolic process [GO:2000988]; negatively regulated by negative regulation of hemicellulose catabolic process [GO:2000989]; positively regulated by GO:2000990 Sources: GOC:mengo_curators Definition: The chemical reactions and pathways resulting in the breakdown of a hemicellulose. Subtypes: xylan catabolic process [GO:0045493], xyloglucan catabolic process [GO:2000899] Also known as: hemicellulose catabolism